{
  "term_label": "nucleoplasm",
  "gene": "UniProtKB:Q8NAG6",
  "term_id": "GO:0005654",
  "gene_symbol": "ANKLE1",
  "gene_name": "Ankyrin repeat and LEM domain-containing protein 1"
}